{
  "term_label": "N-acetylglucosaminylphosphatidylinositol deacetylase activity",
  "gene_symbol": "PIGL",
  "term_id": "GO:0000225",
  "gene_name": "N-acetylglucosaminyl-phosphatidylinositol de-N-acetylase",
  "gene": "UniProtKB:Q9Y2B2"
}